positive regulation of protein localization to early endosome [GO:1902966] (biological process) Relationships: is a type of regulation of protein localization to early endosome [GO:1902965]; is a type of GO:1905668; positively regulates protein localization to early endosome [GO:1902946] Also known as: positive regulation of protein localisation in early endosome, positive regulation of protein localisation to early endosome, positive regulation of protein localization in early endosome, up regulation of protein localisation in early endosome, up regulation of protein localisation to early endosome, up regulation of protein localization in early endosome, up regulation of protein localization to early endosome, up-regulation of protein localisation in early endosome, up-regulation of protein localisation to early endosome, up-regulation of protein localization in early endosome, up-regulation of protein localization to early endosome, upregulation of protein localisation in early endosome, upregulation of protein localisation to early endosome, upregulation of protein localization in early endosome, upregulation of protein localization to early endosome, activation of protein localisation in early endosome, activation of protein localisation to early endosome, activation of protein localization in early endosome, activation of protein localization to early endosome Definition: Any process that activates or increases the frequency, rate or extent of protein localization to early endosome. References: PMID:22621900 Sources: GOC:TermGenie, GOC:sjp, GO_REF:0000058